{
  "term_id": "GO:0006954",
  "term_label": "inflammatory response",
  "gene_name": "Atypical chemokine receptor 1",
  "gene_symbol": "ACKR1",
  "gene": "UniProtKB:Q16570"
}